{
  "gene_symbol": "DUSP21",
  "gene": "UniProtKB:Q9H596",
  "term_id": "UNKNOWN:0002",
  "gene_name": "Dual specificity protein phosphatase 21",
  "term_label": "Unknown biological process"
}